regulation of root morphogenesis [GO:2000067] (biological process) Subtypes: GO:0010061 Relationships: is a type of regulation of plant organ morphogenesis [GO:1905421]; regulates GO:0010015 Definition: Any process that modulates the frequency, rate or extent of root morphogenesis. Sources: GOC:obol